cellular response to insulin-like growth factor stimulus [GO:1990314] (biological process) Definition: Any process that results in a change in state or activity of a cell (in terms of movement, secretion, enzyme production, gene expression, etc.) as a result of an insulin-like growth factor stimulus. References: PMID:20042609 Also known as: cellular response to insulin-like growth factor Relationships: is a type of cellular response to peptide hormone stimulus [GO:0071375]